{
  "gene_name": "FAD-dependent oxidoreductase domain-containing protein 2",
  "term_label": "ERAD pathway",
  "gene": "UniProtKB:Q8IWF2",
  "term_id": "GO:0036503",
  "gene_symbol": "FOXRED2"
}